{
  "gene_name": "Pappalysin-1",
  "gene": "UniProtKB:Q13219",
  "gene_symbol": "PAPPA",
  "term_label": "metalloendopeptidase activity",
  "term_id": "GO:0004222"
}